{
  "gene_name": "RNA-binding protein 6",
  "gene": "UniProtKB:P78332",
  "term_label": "nucleus",
  "term_id": "GO:0005634",
  "gene_symbol": "RBM6"
}